{
  "term_label": "costamere",
  "gene_name": "Small muscular protein",
  "gene": "UniProtKB:Q9UHP9",
  "term_id": "GO:0043034",
  "gene_symbol": "SMPX"
}